{
  "gene": "UniProtKB:Q8TAV4",
  "term_label": "ion channel inhibitor activity",
  "term_id": "GO:0008200",
  "gene_symbol": "STOML3",
  "gene_name": "Stomatin-like protein 3"
}